{
  "term_id": "GO:0032715",
  "gene_symbol": "BPI",
  "gene_name": "Bactericidal permeability-increasing protein",
  "term_label": "negative regulation of interleukin-6 production",
  "gene": "UniProtKB:P17213"
}